regulation of myotome development [GO:2000290] (biological process) Subtypes: positive regulation of myotome development [GO:2000287] Sources: GOC:mah Definition: Any process that modulates the frequency, rate or extent of myotome development. Relationships: is a type of regulation of developmental process [GO:0050793]; regulates myotome development [GO:0061055]